{
  "gene_symbol": "SMAD2",
  "gene": "UniProtKB:Q15796",
  "gene_name": "Mothers against decapentaplegic homolog 2",
  "term_label": "cell differentiation",
  "term_id": "GO:0030154"
}